cephalosporin-C deacetylase activity [GO:0047739] (molecular function) Also known as: cephalosporin C acetyl-esterase activity, cephalosporin C acetyl-hydrolase activity, cephalosporin C acetylase activity, cephalosporin C acetylesterase activity, cephalosporin C deacetylase activity, cephalosporin acetylesterase activity, cephalosporin-C acetylhydrolase activity Sources: EC:3.1.1.41, RHEA:22596 Relationships: is a type of deacetylase activity [GO:0019213]; is a type of carboxylic ester hydrolase activity [GO:0052689] Definition: Catalysis of the reaction: cephalosporin C + H2O = acetate + deacetylcephalosporin C + H+.